{
  "gene_symbol": "BMP5",
  "term_id": "GO:0030509",
  "term_label": "BMP signaling pathway",
  "gene_name": "Bone morphogenetic protein 5",
  "gene": "UniProtKB:P22003"
}